regulation of protein localization to actin cortical patch [GO:1904370] (biological process) Definition: Any process that modulates the frequency, rate or extent of protein localization to actin cortical patch. References: PMID:18216290 Sources: GOC:TermGenie, GO_REF:0000058 Subtypes: GO:1904371, positive regulation of protein localization to actin cortical patch [GO:1904372] Also known as: regulation of protein localisation to actin cortical patch Relationships: is a type of regulation of protein localization to cell cortex [GO:1904776]; regulates protein localization to actin cortical patch [GO:0044379]